mitotic DNA-templated DNA replication [GO:1990506] (biological process) Also known as: mitotic DNA-dependent DNA replication Relationships: is a type of mitotic DNA replication [GO:1902969] Definition: A DNA replication process that uses parental DNA as a template for the DNA-dependent DNA polymerases that synthesize the new strands during the mitotic cell cycle. References: PMID:16120966